{
  "term_id": "GO:0007155",
  "gene_name": "CCN family member 2",
  "term_label": "cell adhesion",
  "gene_symbol": "CCN2",
  "gene": "UniProtKB:P29279"
}